negative regulation of response to tumor cell [GO:0002835] (biological process) Definition: Any process that stops, prevents, or reduces the frequency, rate, or extent of a response to tumor cell. Sources: GOC:add Also known as: down regulation of response to tumor cell, down-regulation of response to tumor cell, downregulation of response to tumor cell, negative regulation of response to tumour cell, inhibition of response to tumor cell Relationships: is a type of GO:0002832; is_a GO:0002834; negatively regulates response to tumor cell [GO:0002347] Subtypes: negative regulation of immune response to tumor cell [GO:0002838]